{
  "gene_name": "Follistatin-related protein 3",
  "term_id": "GO:0005615",
  "term_label": "extracellular space",
  "gene_symbol": "FSTL3",
  "gene": "UniProtKB:O95633"
}